{
  "term_id": "UNKNOWN:0003",
  "gene": "UniProtKB:Q9Y3Q0",
  "term_label": "Unknown cellular component",
  "gene_name": "N-acetylated-alpha-linked acidic dipeptidase 2",
  "gene_symbol": "NAALAD2"
}